{
  "term_label": "negative regulation of transcription by RNA polymerase II",
  "gene_symbol": "MAGEA3",
  "gene_name": "Melanoma-associated antigen 3",
  "term_id": "GO:0000122",
  "gene": "UniProtKB:P43357"
}